{
  "term_label": "nitric-oxide synthase activity",
  "gene_name": "Nitric oxide synthase 1",
  "gene_symbol": "NOS1",
  "gene": "UniProtKB:P29475",
  "term_id": "GO:0004517"
}